negative regulation of transcription by RNA polymerase I [GO:0016479] (biological process) Relationships: is a type of GO:0006356; is a type of GO:0045892; negatively regulates transcription by RNA polymerase I [GO:0006360] Subtypes: negative regulation of transcription of nucleolar large rRNA by RNA polymerase I [GO:1901837], negative regulation of termination of RNA polymerase I transcription [GO:2000731], negative regulation of transcription elongation by RNA polymerase I [GO:2001208] Definition: Any process that stops, prevents, or reduces the frequency, rate or extent of transcription mediated by RNA polymerase I. Sources: GOC:go_curators Also known as: down regulation of transcription from RNA polymerase I promoter, down-regulation of transcription from RNA polymerase I promoter, downregulation of transcription from RNA polymerase I promoter, negative regulation of transcription from Pol I promoter, negative regulation of transcription from RNA polymerase I promoter, inhibition of transcription from RNA polymerase I promoter